{
  "term_id": "GO:0005634",
  "gene_symbol": "ZNF770",
  "gene": "UniProtKB:Q6IQ21",
  "term_label": "nucleus",
  "gene_name": "Zinc finger protein 770"
}